{
  "gene": "UniProtKB:Q5XKR4",
  "term_id": "GO:0030182",
  "gene_name": "Homeobox protein orthopedia",
  "gene_symbol": "OTP",
  "term_label": "neuron differentiation"
}